{
  "gene": "UniProtKB:O43516",
  "gene_symbol": "WIPF1",
  "gene_name": "WAS_WASL-interacting protein family member 1",
  "term_id": "UNKNOWN:0001",
  "term_label": "Unknown molecular function"
}